{
  "gene_symbol": "PMP22",
  "gene_name": "Peripheral myelin protein 22",
  "term_id": "UNKNOWN:0001",
  "term_label": "Unknown molecular function",
  "gene": "UniProtKB:Q01453"
}